{
  "gene": "UniProtKB:O75916",
  "term_id": "GO:0005737",
  "gene_name": "Regulator of G-protein signaling 9",
  "term_label": "cytoplasm",
  "gene_symbol": "RGS9"
}